{
  "gene": "UniProtKB:O43707",
  "term_id": "GO:0042995",
  "gene_name": "Alpha-actinin-4",
  "term_label": "cell projection",
  "gene_symbol": "ACTN4"
}